thrombopoietin-mediated signaling pathway [GO:0038163] (biological process) References: PMID:19630807 Sources: GOC:nhn, GOC:signaling Relationships: is a type of chemokine-mediated signaling pathway [GO:0070098] Also known as: THPO signaling pathway, THPO/MPL signaling pathway, thrombopoietin receptor signaling pathway Definition: The series of molecular signals initiated by thrombopoietin binding to its receptor on the surface of a target cell, and ending with the regulation of a downstream cellular process, e.g. transcription.